{
  "gene_symbol": "DUX3",
  "term_id": "GO:0005634",
  "gene_name": "Putative double homeobox protein 3",
  "term_label": "nucleus",
  "gene": "UniProtKB:Q96PT4"
}